{
  "term_id": "GO:0005634",
  "gene_symbol": "SIX2",
  "gene_name": "Homeobox protein SIX2",
  "gene": "UniProtKB:Q9NPC8",
  "term_label": "nucleus"
}